{
  "gene_symbol": "TBC1D21",
  "term_id": "GO:0048227",
  "term_label": "plasma membrane to endosome transport",
  "gene_name": "TBC1 domain family member 21",
  "gene": "UniProtKB:Q8IYX1"
}